{
  "gene_symbol": "YPEL4",
  "gene_name": "Protein yippee-like 4",
  "term_label": "Unknown molecular function",
  "term_id": "UNKNOWN:0001",
  "gene": "UniProtKB:Q96NS1"
}